negative regulation of leukocyte proliferation [GO:0070664] (biological process) Definition: Any process that stops, prevents, or reduces the frequency, rate or extent of leukocyte proliferation. Also known as: down regulation of leukocyte proliferation, down-regulation of leukocyte proliferation, downregulation of leukocyte proliferation, inhibition of leukocyte proliferation Sources: GOC:add, GOC:mah Subtypes: negative regulation of mononuclear cell proliferation [GO:0032945], negative regulation of mast cell proliferation [GO:0070667], GO:0090291, negative regulation of macrophage proliferation [GO:0120042] Relationships: is a type of negative regulation of cell population proliferation [GO:0008285]; is a type of regulation of leukocyte proliferation [GO:0070663]; negatively regulates GO:0070661